{
  "gene_name": "Cadherin-10",
  "gene_symbol": "CDH10",
  "term_id": "GO:0045296",
  "gene": "UniProtKB:Q9Y6N8",
  "term_label": "cadherin binding"
}